flavone synthase activity [GO:0033759] (molecular function) Definition: Catalysis of the reaction: a flavanone + 2-oxoglutarate + O2 = a flavone + succinate + CO2 + H2O. Relationships: is a type of 2-oxoglutarate-dependent dioxygenase activity [GO:0016706]; is part of GO:0051553 Sources: EC:1.14.20.5 Also known as: FNS I, flavanone,2-oxoglutarate:oxygen oxidoreductase (dehydrating) activity, flavone synthase I activity